lovastatin biosynthetic process [GO:0140735] (BP) Definition: The chemical reactions and pathways resulting in the formation of lovastatin (also known as mevinolin, mevacor or monacolin K), a hypolipidemic inhibitor of (3S)-hydroxymethylglutaryl-coenzyme A (HMG-CoA) reductase (HMGR). Also known as: lovastatin anabolism, lovastatin biosynthesis, lovastatin formation, lovastatin synthesis, mevacor anabolism, mevacor biosynthesis, mevacor biosynthetic process, mevacor formation, mevacor synthesis, mevinolin anabolism, mevinolin biosynthesis, mevinolin biosynthetic process, mevinolin formation,, mevinolin synthesis, monacolin K anabolism, monacolin K biosynthesis, monacolin K biosynthetic process, monacolin K formation, monacolin K synthesis References: PMID:10334994, PMID:10381407 Regulation: positively regulated by GO:0140736 Relationships: is a type of polyketide biosynthetic process [GO:0030639]; is a type of mycotoxin biosynthetic process [GO:0043386]; is_a lactone biosynthetic process [GO:1901336]; is a type of fatty acid derivative biosynthetic process [GO:1901570]